{
  "gene": "UniProtKB:Q6ZRF7",
  "term_label": "Unknown molecular function",
  "term_id": "UNKNOWN:0001",
  "gene_symbol": "ZNF818P",
  "gene_name": "Putative zinc finger protein 818"
}